negative regulation of establishment or maintenance of bipolar cell polarity regulating cell shape [GO:2000750] (biological process) Definition: Any process that stops, prevents or reduces the frequency, rate or extent of establishment or maintenance of bipolar cell polarity regulating cell shape. Sources: GOC:mah Relationships: is a type of regulation of establishment or maintenance of bipolar cell polarity regulating cell shape [GO:2000100]; is a type of negative regulation of establishment or maintenance of cell polarity regulating cell shape [GO:2000770]; RO_0002212 establishment or maintenance of bipolar cell polarity regulating cell shape [GO:0061246] Subtypes: GO:0061362